Schmidt-Lanterman incisure [GO:0043220] (cellular component) Definition: Regions within compact myelin in which the cytoplasmic faces of the enveloping myelin sheath are not tightly juxtaposed, and include cytoplasm from the cell responsible for making the myelin. Schmidt-Lanterman incisures occur in the compact myelin internode, while lateral loops are analogous structures found in the paranodal region adjacent to the nodes of Ranvier. Relationships: is a type of GO:0110165; is part of compact myelin [GO:0043218] Also known as: Schmidt-Lanterman cleft Sources: GOC:dgh